{
  "gene_symbol": "PDLIM7",
  "term_label": "actin binding",
  "gene_name": "PDZ and LIM domain protein 7",
  "term_id": "GO:0003779",
  "gene": "UniProtKB:Q9NR12"
}